{
  "term_label": "Unknown molecular function",
  "gene_symbol": "TMEFF2",
  "gene_name": "Tomoregulin-2",
  "gene": "UniProtKB:Q9UIK5",
  "term_id": "UNKNOWN:0001"
}